{
  "gene_name": "Immunoglobulin heavy variable 4-61",
  "term_label": "antigen binding",
  "gene_symbol": "IGHV4-61",
  "term_id": "GO:0003823",
  "gene": "UniProtKB:A0A0C4DH41"
}